chloroplast ADPG pyrophosphorylase complex [GO:0030933] (cellular component) Definition: An ADPG pyrophosphorylase complex found in the chloroplast. Sources: GOC:mah Relationships: is a type of plastid ADPG pyrophosphorylase complex [GO:0031009]; is part of GO:0009507